archaeal proton-transporting A-type ATPase complex [GO:1990490] (cellular component) Relationships: is a type of proton-transporting two-sector ATPase complex [GO:0016469]; is a type of ATPase complex [GO:1904949] References: PMID:15473999, PMID:24650628 Sources: GOC:mengo_curators Also known as: A-type ATPase protein complex, archaeal A-type ATPase protein complex Definition: A large proton-transporting two-sector ATPase protein complex that catalyzes the synthesis or hydrolysis of ATP by a rotational mechanism, coupled to the transport of protons across a membrane and is found in Archaea.